{
  "gene": "UniProtKB:Q8TDI7",
  "term_id": "GO:0008381",
  "term_label": "mechanosensitive monoatomic ion channel activity",
  "gene_symbol": "TMC2",
  "gene_name": "Transmembrane channel-like protein 2"
}